{
  "term_label": "Unknown molecular function",
  "gene_name": "Stabilin-1",
  "gene": "UniProtKB:Q9NY15",
  "term_id": "UNKNOWN:0001",
  "gene_symbol": "STAB1"
}